{
  "term_label": "external side of plasma membrane",
  "gene": "UniProtKB:P12318",
  "gene_symbol": "FCGR2A",
  "term_id": "GO:0009897",
  "gene_name": "Low affinity immunoglobulin gamma Fc region receptor II-a"
}